precorrin-6A synthase (deacetylating) activity [GO:0043819] (molecular function) Definition: Catalysis of the reaction: S-adenosyl-L-methionine + H2O + precorrin-5 = S-adenosyl-L-homocysteine + acetate + 2 H+ + precorrin-6X. Sources: EC:2.1.1.152, RHEA:18261 Also known as: S-adenosyl-L-methionine:precorrin-5 C1-methyltransferase (deacetylating), CobF, precorrin-6X synthase (deacetylating) activity Relationships: is a type of methyltransferase activity [GO:0008168]